{
  "gene_name": "Interferon-induced protein with tetratricopeptide repeats 3",
  "gene": "UniProtKB:O14879",
  "gene_symbol": "IFIT3",
  "term_label": "cytosol",
  "term_id": "GO:0005829"
}